tRNA-dihydrouridine47 synthase activity [GO:0102265] (molecular function) Relationships: is a type of tRNA dihydrouridine synthase activity [GO:0017150] Sources: EC:1.3.1.89, GOC:pz Definition: Catalysis of the reaction: a 5,6-dihydrouracil47 in tRNA + NAD(P) = H+ + a uracil47 in tRNA + NAD(P)H.